{
  "gene_symbol": "SLC16A12",
  "term_label": "plasma membrane",
  "term_id": "GO:0005886",
  "gene_name": "Monocarboxylate transporter 12",
  "gene": "UniProtKB:Q6ZSM3"
}